positive regulation of vascular associated smooth muscle contraction [GO:1904695] (BP) Definition: Any process that activates or increases the frequency, rate or extent of vascular smooth muscle contraction. References: PMID:22158624 Sources: GOC:BHF, GOC:BHF_miRNA, GOC:TermGenie, GOC:rph, GO_REF:0000058 Also known as: positive regulation of vascular smooth muscle contraction, up regulation of vascular smooth muscle contraction, up-regulation of vascular smooth muscle contraction, upregulation of vascular smooth muscle contraction, activation of vascular smooth muscle contraction Relationships: is a type of GO:0003056; is a type of positive regulation of vasoconstriction [GO:0045907]; is a type of GO:0045987; RO_0002213 GO:0014829 Subtypes: GO:0062087, positive regulation of artery smooth muscle contraction [GO:1905656]